{
  "gene": "UniProtKB:Q86SG6",
  "term_label": "protein serine/threonine kinase activity",
  "term_id": "GO:0004674",
  "gene_symbol": "NEK8",
  "gene_name": "Serine_threonine-protein kinase Nek8"
}